{
  "gene": "UniProtKB:Q8NHS0",
  "term_label": "cytoplasm",
  "gene_symbol": "DNAJB8",
  "gene_name": "DnaJ homolog subfamily B member 8",
  "term_id": "GO:0005737"
}